regulation of eosinophil activation [GO:1902566] (biological process) Definition: Any process that modulates the frequency, rate or extent of eosinophil activation. References: PMID:16254138 Sources: GOC:TermGenie Relationships: is a type of regulation of leukocyte activation [GO:0002694]; regulates eosinophil activation [GO:0043307] Subtypes: negative regulation of eosinophil activation [GO:1902567], positive regulation of eosinophil activation [GO:1902568]